{
  "gene": "UniProtKB:P43220",
  "term_id": "GO:0044508",
  "term_label": "glucagon-like peptide 1 receptor activity",
  "gene_symbol": "GLP1R",
  "gene_name": "Glucagon-like peptide 1 receptor"
}